catecholamine uptake [GO:0090493] (biological process) Subtypes: norepinephrine uptake [GO:0051620], catecholamine uptake involved in synaptic transmission [GO:0051934], dopamine uptake [GO:0090494] Sources: GOC:dph, GOC:tb Relationships: is a type of GO:0051937 Definition: The directed movement of catecholamine into a cell.